{
  "term_id": "GO:0048278",
  "gene": "UniProtKB:O14662",
  "gene_name": "Syntaxin-16",
  "term_label": "vesicle docking",
  "gene_symbol": "STX16"
}